{
  "gene_name": "Matrix metalloproteinase-19",
  "gene": "UniProtKB:Q99542",
  "term_label": "extracellular space",
  "term_id": "GO:0005615",
  "gene_symbol": "MMP19"
}